{
  "gene_name": "Transketolase-like protein 1",
  "term_label": "transketolase activity",
  "term_id": "GO:0004802",
  "gene": "UniProtKB:P51854",
  "gene_symbol": "TKTL1"
}